microsatellite binding [GO:0035939] (molecular function) References: PMID:21290414 Sources: GOC:yaf, SO:0000289 Also known as: VNTR binding, microsatellite DNA binding, variable number tandem repeat binding Relationships: is a type of satellite DNA binding [GO:0003696] Definition: Binding to a microsatellite, a repeat_region in DNA containing repeat units (2 to 4 base pairs) that is repeated multiple times in tandem.